{
  "gene": "UniProtKB:Q96GW9",
  "gene_name": "Methionine--tRNA ligase, mitochondrial",
  "term_label": "mitochondrion",
  "gene_symbol": "MARS2",
  "term_id": "GO:0005739"
}